response to forskolin [GO:1904321] (biological process) References: PMID:15937517 Sources: GOC:TermGenie, GO_REF:0000071 Subtypes: cellular response to forskolin [GO:1904322] Definition: Any process that results in a change in state or activity of a cell or an organism (in terms of movement, secretion, enzyme production, gene expression, etc.) as a result of a forskolin stimulus. Relationships: is a type of GO:0033993; is a type of response to alcohol [GO:0097305]; is a type of GO:1901654